{
  "gene_name": "Ubiquitin carboxyl-terminal hydrolase MINDY-2",
  "gene": "UniProtKB:Q8NBR6",
  "term_label": "Unknown biological process",
  "gene_symbol": "MINDY2",
  "term_id": "UNKNOWN:0002"
}